regulation of cardiac chamber morphogenesis [GO:1901219] (biological process) Sources: GOC:BHF, GOC:TermGenie Also known as: regulation of heart chamber morphogenesis Definition: Any process that modulates the frequency, rate or extent of cardiac chamber morphogenesis. Subtypes: negative regulation of cardiac chamber morphogenesis [GO:1901220], positive regulation of cardiac chamber morphogenesis [GO:1901221] Relationships: is a type of GO:2000826; regulates cardiac chamber morphogenesis [GO:0003206]